{
  "term_label": "regulation of signal transduction",
  "term_id": "GO:0009966",
  "gene": "UniProtKB:O43815",
  "gene_name": "Striatin",
  "gene_symbol": "STRN"
}